{
  "gene_name": "Protein naked cuticle homolog 1",
  "gene_symbol": "NKD1",
  "gene": "UniProtKB:Q969G9",
  "term_id": "UNKNOWN:0001",
  "term_label": "Unknown molecular function"
}